{
  "gene": "UniProtKB:Q969Y2",
  "term_label": "Unknown molecular function",
  "term_id": "UNKNOWN:0001",
  "gene_symbol": "GTPBP3",
  "gene_name": "tRNA modification GTPase GTPBP3, mitochondrial"
}